{
  "gene": "UniProtKB:P30532",
  "term_label": "acetylcholine receptor signaling pathway",
  "term_id": "GO:0095500",
  "gene_symbol": "CHRNA5",
  "gene_name": "Neuronal acetylcholine receptor subunit alpha-5"
}